{
  "gene_symbol": "BOP1",
  "term_id": "GO:0070545",
  "term_label": "PeBoW complex",
  "gene_name": "Ribosome biogenesis protein BOP1",
  "gene": "UniProtKB:Q14137"
}